response to freezing [GO:0050826] (biological process) Definition: Any process that results in a change in state or activity of a cell or an organism (in terms of movement, secretion, enzyme production, gene expression, etc.) as a result of a freezing stimulus, temperatures below 0 degrees Celsius. Sources: GOC:jl Subtypes: cellular response to freezing [GO:0071497] Relationships: is a type of response to cold [GO:0009409] Also known as: antifreeze activity, ice nucleation inhibitor activity